{
  "term_label": "Unknown molecular function",
  "gene_name": "Protein FAM201A",
  "term_id": "UNKNOWN:0001",
  "gene": "UniProtKB:Q5SY85",
  "gene_symbol": "FAM201A"
}